{
  "gene": "UniProtKB:Q5VZR4",
  "term_id": "UNKNOWN:0001",
  "gene_name": "Major facilitator superfamily domain-containing 14C pseudogene",
  "gene_symbol": "MFSD14CP",
  "term_label": "Unknown molecular function"
}